negative regulation of endocardial cushion to mesenchymal transition [GO:0140050] (biological process) Relationships: is a type of negative regulation of cardiac epithelial to mesenchymal transition [GO:0062044]; is a type of regulation of endocardial cushion to mesenchymal transition [GO:0140049]; negatively regulates GO:0090500 Subtypes: negative regulation of endocardial cushion to mesenchymal transition involved in heart valve formation [GO:2000801] References: PMID:21778427 Sources: GOC:BHF, GOC:BHF_miRNA, GOC:rph Definition: Any process that stops, prevents or reduces the frequency, rate or extent of endocardial cushion to mesenchymal transition.